negative regulation of macromolecule biosynthetic process [GO:0010558] (biological process) Sources: GOC:dph, GOC:tb Relationships: is a type of negative regulation of biosynthetic process [GO:0009890]; is a type of regulation of macromolecule biosynthetic process [GO:0010556]; is a type of negative regulation of macromolecule metabolic process [GO:0010605]; negatively regulates macromolecule biosynthetic process [GO:0009059] Definition: Any process that decreases the rate, frequency or extent of the chemical reactions and pathways resulting in the formation of a macromolecule, any molecule of high relative molecular mass, the structure of which essentially comprises the multiple repetition of units derived, actually or conceptually, from molecules of low relative molecular mass. Subtypes: negative regulation of glycoprotein biosynthetic process [GO:0010561], negative regulation of gene expression [GO:0010629], negative regulation of MHC class I biosynthetic process [GO:0045344], GO:0045347, negative regulation of glycogen biosynthetic process [GO:0045719], negative regulation of integrin biosynthetic process [GO:0045720], GO:0046986, GO:0060636, negative regulation of hyaluronan biosynthetic process [GO:1900126], negative regulation of cutin biosynthetic process [GO:1901958], GO:1902679, negative regulation of protein lipidation [GO:1903060], negative regulation of DNA biosynthetic process [GO:2000279], GO:2001007, GO:7770012